{
  "gene": "UniProtKB:Q96S15",
  "gene_name": "GATOR complex protein WDR24",
  "term_label": "vacuolar membrane",
  "term_id": "GO:0005774",
  "gene_symbol": "WDR24"
}